{
  "term_id": "GO:0014704",
  "gene": "UniProtKB:P78310",
  "gene_name": "Coxsackievirus and adenovirus receptor",
  "gene_symbol": "CXADR",
  "term_label": "intercalated disc"
}